{
  "gene_name": "C5a anaphylatoxin chemotactic receptor 1",
  "term_label": "G protein-coupled receptor activity",
  "gene_symbol": "C5AR1",
  "gene": "UniProtKB:P21730",
  "term_id": "GO:0004930"
}